{
  "term_label": "endogenous lipid antigen binding",
  "gene_symbol": "CD1D",
  "gene_name": "Antigen-presenting glycoprotein CD1d",
  "term_id": "GO:0030883",
  "gene": "UniProtKB:P15813"
}